{
  "gene": "UniProtKB:A6NM45",
  "term_id": "GO:0005923",
  "term_label": "bicellular tight junction",
  "gene_name": "Putative claudin-24",
  "gene_symbol": "CLDN24"
}